{
  "gene": "UniProtKB:Q9NSD5",
  "gene_symbol": "SLC6A13",
  "term_id": "GO:0006865",
  "gene_name": "Sodium- and chloride-dependent GABA transporter 2",
  "term_label": "amino acid transport"
}